{
  "term_id": "GO:0000786",
  "gene_name": "Histone H2B type 1-K",
  "gene_symbol": "H2BC12",
  "gene": "UniProtKB:O60814",
  "term_label": "nucleosome"
}